{
  "gene_name": "Protein SSX1",
  "gene": "UniProtKB:Q16384",
  "gene_symbol": "SSX1",
  "term_label": "Unknown biological process",
  "term_id": "UNKNOWN:0002"
}